{
  "gene_symbol": "SFT2D3",
  "term_id": "UNKNOWN:0002",
  "gene_name": "Vesicle transport protein SFT2C",
  "term_label": "Unknown biological process",
  "gene": "UniProtKB:Q587I9"
}